adaptation to pheromone regulating conjugation with mutual genetic exchange [GO:0000760] (biological process) Relationships: is a type of response to pheromone regulating conjugation with mutual genetic exchange [GO:0000756]; is a type of negative adaptation of signaling pathway [GO:0022401]; is a type of regulation of reproductive process [GO:2000241] Sources: GOC:clt Also known as: desensitization to pheromone during conjugation without cellular fusion, adaptation to pheromone involved conjugation without cellular fusion Definition: In organisms that undergo conjugation without cellular fusion, the process resulting in desensitization following exposure to pheromone stimulus that act to down-regulate further stimulation or block initial conjugation responses.